{
  "term_label": "detection of chemical stimulus involved in sensory perception of smell",
  "gene": "UniProtKB:Q8NH81",
  "gene_name": "Olfactory receptor 10G6",
  "gene_symbol": "OR10G6",
  "term_id": "GO:0050911"
}